negative regulation of butyryl-CoA catabolic process to butanol [GO:1900498] (biological process) Relationships: is a type of negative regulation of amide metabolic process [GO:0034249]; is_a negative regulation of fatty acid metabolic process [GO:0045922]; is_a negative regulation of nucleobase-containing compound metabolic process [GO:0045934]; is a type of negative regulation of phosphate metabolic process [GO:0045936]; is a type of GO:0050995; is a type of negative regulation of lipid biosynthetic process [GO:0051055]; is a type of GO:1900497; is a type of negative regulation of alcohol biosynthetic process [GO:1902931]; negatively regulates butyryl-CoA catabolic process to butanol [GO:0044582] Also known as: down regulation of butyryl-CoA catabolic process to butanol, down regulation of butyryl-CoA catabolism to butanol, down-regulation of butyryl-CoA catabolic process to butanol, down-regulation of butyryl-CoA catabolism to butanol, downregulation of butyryl-CoA catabolic process to butanol, downregulation of butyryl-CoA catabolism to butanol, inhibition of butyryl-CoA catabolism to butanol, negative regulation of butyryl-CoA catabolism to butanol, inhibition of butyryl-CoA catabolic process to butanol Definition: Any process that stops, prevents or reduces the frequency, rate or extent of butyryl-CoA catabolic process to butanol. Sources: GOC:TermGenie, GOC:mengo_curators